{
  "term_label": "cysteine-type deubiquitinase activity",
  "gene_symbol": "USP14",
  "term_id": "GO:0004843",
  "gene": "UniProtKB:P54578",
  "gene_name": "Ubiquitin carboxyl-terminal hydrolase 14"
}